nicotinic acid receptor activity [GO:0070553] (molecular function) Also known as: niacin receptor activity Relationships: is a type of G protein-coupled receptor activity [GO:0004930] References: PMID:12522134 Sources: GOC:mah Definition: Combining with nicotinic acid to initiate a change in cell activity.